{
  "gene_name": "AF4_FMR2 family member 1",
  "gene": "UniProtKB:P51825",
  "term_label": "super elongation complex",
  "term_id": "GO:0032783",
  "gene_symbol": "AFF1"
}